{
  "gene": "UniProtKB:A0A0B4J1V2",
  "term_label": "Unknown cellular component",
  "gene_name": "Immunoglobulin heavy variable 2-26",
  "term_id": "UNKNOWN:0003",
  "gene_symbol": "IGHV2-26"
}